{
  "term_id": "UNKNOWN:0003",
  "gene_name": "Zinc finger protein 707",
  "gene": "UniProtKB:Q96C28",
  "gene_symbol": "ZNF707",
  "term_label": "Unknown cellular component"
}